positive regulation of penicillin biosynthetic process [GO:1900198] (biological process) Relationships: is a type of positive regulation of penicillin metabolic process [GO:0033246]; is a type of GO:1900196; is a type of positive regulation of secondary metabolite biosynthetic process [GO:1900378]; positively regulates penicillin biosynthetic process [GO:0042318] Sources: GOC:TermGenie, GOC:di Also known as: activation of penicillin anabolism, activation of penicillin biosynthesis, activation of penicillin formation, activation of penicillin synthesis, positive regulation of penicillin anabolism, positive regulation of penicillin biosynthesis, positive regulation of penicillin formation, positive regulation of penicillin synthesis, up regulation of penicillin anabolism, up regulation of penicillin biosynthesis, up regulation of penicillin biosynthetic process, up regulation of penicillin formation, up regulation of penicillin synthesis, up-regulation of penicillin anabolism, up-regulation of penicillin biosynthesis, up-regulation of penicillin biosynthetic process, up-regulation of penicillin formation, up-regulation of penicillin synthesis, upregulation of penicillin anabolism, upregulation of penicillin biosynthesis, upregulation of penicillin biosynthetic process, upregulation of penicillin formation, upregulation of penicillin synthesis, activation of penicillin biosynthetic process Definition: Any process that activates or increases the frequency, rate or extent of penicillin biosynthetic process.